{
  "gene_name": "Histone-lysine N-methyltransferase SETDB2",
  "gene": "UniProtKB:Q96T68",
  "gene_symbol": "SETDB2",
  "term_id": "GO:0010629",
  "term_label": "negative regulation of gene expression"
}